{
  "gene": "UniProtKB:Q9UGL9",
  "gene_symbol": "CRCT1",
  "term_id": "UNKNOWN:0001",
  "term_label": "Unknown molecular function",
  "gene_name": "Cysteine-rich C-terminal protein 1"
}